platelet-derived growth factor receptor-beta signaling pathway [GO:0035791] (biological process) Also known as: PDGF receptor-beta signaling pathway, PDGFR-beta signaling pathway, betaPDGF receptor signaling pathway, platelet-derived growth factor receptor-beta signalling pathway Subtypes: VEGF-activated platelet-derived growth factor receptor-beta signaling pathway [GO:0038088], regulation of metanephric mesenchymal cell migration by platelet-derived growth factor receptor-beta signaling pathway [GO:1900238] Definition: The series of molecular signals initiated by the binding of a ligand to a beta-type platelet-derived growth factor receptor (PDGFbeta) on the surface of a signal-receiving cell, and ending with the regulation of a downstream cellular process, e.g. transcription. References: PMID:10372961 Sources: GOC:bf, GOC:signaling, GOC:yaf Regulation: regulated by regulation of platelet-derived growth factor receptor-beta signaling pathway [GO:2000586]; RO_0002212 by negative regulation of platelet-derived growth factor receptor-beta signaling pathway [GO:2000587]; positively regulated by GO:2000588 Relationships: is a type of platelet-derived growth factor receptor signaling pathway [GO:0048008]